{
  "gene": "UniProtKB:O95400",
  "gene_name": "CD2 antigen cytoplasmic tail-binding protein 2",
  "term_label": "U5 snRNP",
  "term_id": "GO:0005682",
  "gene_symbol": "CD2BP2"
}